{
  "term_id": "GO:0005743",
  "gene": "UniProtKB:Q9Y5U8",
  "gene_symbol": "MPC1",
  "term_label": "mitochondrial inner membrane",
  "gene_name": "Mitochondrial pyruvate carrier 1"
}